interleukin-10 receptor complex [GO:1905571] (cellular component) Relationships: is a type of receptor complex [GO:0043235] References: PMID:16982608 Sources: GOC:TermGenie, GOC:bhm, GO_REF:0000088 Note: An example of this is IL10RA in human (UniProt symbol Q13651) in PMID:16982608 (inferred from physical interaction). Also known as: IL-10 receptor complex, IL-10-receptor complex, IL10 receptor complex, interleukin-10-receptor complex Definition: A protein complex that binds interleukin-10 (IL-10) and that consists of, at a minimum, a dimeric interleukin, an alpha and a beta chain as well as optional additional kinase subunits. The alpha chain binds IL-10 with high affinity and subsequently binds the common beta receptor chain that forms part of multiple interleukin receptors.